mitochondrial fusion [GO:0008053] (biological process) Regulation: regulated by GO:0010635; positively regulated by GO:0010636; negatively regulated by negative regulation of mitochondrial fusion [GO:0010637] Relationships: is a type of mitochondrion organization [GO:0007005]; is a type of organelle fusion [GO:0048284] Also known as: mitochondrion fusion, mitochondrial membrane fusion Subtypes: GO:1990046 Definition: Merging of two or more mitochondria within a cell to form a single compartment. References: PMID:11038192, PMID:12052774